dihydrofolic acid binding [GO:0051871] (molecular function) Also known as: DHF binding, dihydrofolate binding Sources: ISBN:0721662544 Relationships: is a type of GO:0031406; is a type of GO:0072341; is a type of heterocyclic compound binding [GO:1901363] Definition: Binding to dihydrofolic acid, a folic acid in which the bicyclic pteridine structure is in the dihydro, partially reduced form; they are intermediates in folate metabolism and are reduced to their tetrahydro, reduced forms.